{
  "term_label": "nucleus",
  "gene_symbol": "DPRX",
  "term_id": "GO:0005634",
  "gene": "UniProtKB:A6NFQ7",
  "gene_name": "Divergent paired-related homeobox"
}